{
  "gene_symbol": "NDFIP2",
  "term_label": "endoplasmic reticulum",
  "term_id": "GO:0005783",
  "gene_name": "NEDD4 family-interacting protein 2",
  "gene": "UniProtKB:Q9NV92"
}